dibenzo-p-dioxin catabolic process [GO:0019341] (biological process) Also known as: dibenzo-p-dioxin breakdown, dibenzo-p-dioxin catabolism, dibenzo-p-dioxin degradation Definition: The chemical reactions and pathways resulting in the breakdown of dibenzo-p-dioxin, a substance composed of two benzene rings linked by two ether bonds. Sources: GOC:ai Relationships: is a type of dibenzo-p-dioxin metabolic process [GO:0018894]; is a type of xenobiotic catabolic process [GO:0042178]; is a type of small molecule catabolic process [GO:0044282]